{
  "term_id": "GO:0005764",
  "gene": "UniProtKB:P51151",
  "gene_name": "Ras-related protein Rab-9A",
  "gene_symbol": "RAB9A",
  "term_label": "lysosome"
}